negative regulation of B cell cytokine production [GO:0002722] (biological process) Definition: Any process that stops, prevents, or reduces the frequency, rate, or extent of B cell cytokine production. Sources: GOC:add Also known as: down regulation of B cell cytokine production, down-regulation of B cell cytokine production, downregulation of B cell cytokine production, negative regulation of B lymphocyte cytokine production, negative regulation of B-cell cytokine production, negative regulation of B-lymphocyte cytokine production, inhibition of B cell cytokine production Relationships: is a type of GO:0002713; is a type of negative regulation of cytokine production involved in immune response [GO:0002719]; is a type of regulation of B cell cytokine production [GO:0002721]; negatively regulates B cell cytokine production [GO:0002368]